{
  "term_id": "GO:0000981",
  "gene_name": "Upstream stimulatory factor 1",
  "gene_symbol": "USF1",
  "term_label": "DNA-binding transcription factor activity, RNA polymerase II-specific",
  "gene": "UniProtKB:P22415"
}